{
  "term_id": "GO:0005975",
  "gene_name": "Alpha-amylase 1B",
  "gene": "UniProtKB:P0DTE7",
  "gene_symbol": "AMY1B",
  "term_label": "carbohydrate metabolic process"
}